cyanidin 3-O-glucoside metabolic process [GO:1901038] (biological process) Subtypes: cyanidin 3-O-glucoside biosynthetic process [GO:0033485] Relationships: is a type of flavonoid metabolic process [GO:0009812]; is a type of glycoside metabolic process [GO:0016137] Also known as: cyanidin 3-O-beta-D-glucoside metabolic process, cyanidin 3-O-beta-D-glucoside metabolism References: PMID:21899608 Sources: GOC:TermGenie Definition: The chemical reactions and pathways involving cyanidin 3-O-beta-D-glucoside.